post-transcriptional regulation of gene expression [GO:0010608] (biological process) Subtypes: regulation of translation [GO:0006417], mRNA localization resulting in post-transcriptional regulation of gene expression [GO:0010609], post-transcriptional gene silencing [GO:0016441], regulation of RNA stability [GO:0043487] Also known as: posttranscriptional regulation of gene expression Definition: Any process that modulates the frequency, rate or extent of gene expression after the production of an RNA transcript. Sources: GOC:dph, GOC:tb Relationships: is a type of regulation of gene expression [GO:0010468]